{
  "gene_symbol": "MEIKIN",
  "gene_name": "Meiosis-specific kinetochore protein",
  "term_label": "homologous chromosome segregation",
  "gene": "UniProtKB:A0A087WXM9",
  "term_id": "GO:0045143"
}